peptide butyryltransferase activity [GO:0140065] (molecular function) Definition: Catalysis of the reaction: butyryl-CoA + lysine in peptide = CoA + N-butyryl-lysine-peptide. Subtypes: histone butyryltransferase activity [GO:0140069] References: PMID:27105113 Also known as: protein butyryltransferase activity Relationships: is a type of N-acyltransferase activity [GO:0016410]